{
  "gene_name": "Interferon-stimulated gene 20 kDa protein",
  "term_id": "GO:0006308",
  "gene_symbol": "ISG20",
  "term_label": "DNA catabolic process",
  "gene": "UniProtKB:Q96AZ6"
}